xenobiotic transmembrane transport [GO:0006855] (biological process) Also known as: drug membrane transport, drug transmembrane transport, multidrug transport Sources: GOC:ai, GOC:bf, GOC:krc Definition: The process in which a xenobiotic, a compound foreign to the organism exposed to it, is transported across a membrane. It may be synthesized by another organism (like ampicilin) or it can be a synthetic chemical. Relationships: is a type of GO:0042908; is a type of transmembrane transport [GO:0055085] Note: Note that this term is not intended for use in annotating lateral movement within membranes.